{
  "gene_name": "Chromosome transmission fidelity protein 18 homolog",
  "gene_symbol": "CHTF18",
  "term_label": "Unknown biological process",
  "gene": "UniProtKB:Q8WVB6",
  "term_id": "UNKNOWN:0002"
}